raffinose transport [GO:0015773] (biological process) Definition: The directed movement of raffinose into, out of or within a cell, or between cells, by means of some agent such as a transporter or pore. Raffinose occurs in plants almost as commonly as sucrose and is present in cereal grains, cotton seeds, and many legumes. It is synthesized from sucrose by transfer of a galactopyranoside from myo-inositol. Sources: ISBN:0198506732 Relationships: is a type of trisaccharide transport [GO:2001088]